{
  "gene": "UniProtKB:Q9GZN0",
  "term_id": "GO:0007602",
  "gene_name": "Probable G-protein coupled receptor 88",
  "gene_symbol": "GPR88",
  "term_label": "phototransduction"
}